{
  "gene_name": "Nucleoside diphosphate kinase, mitochondrial",
  "term_id": "UNKNOWN:0003",
  "gene_symbol": "NME4",
  "term_label": "Unknown cellular component",
  "gene": "UniProtKB:O00746"
}